{
  "gene_symbol": "SEPTIN3",
  "gene_name": "Neuronal-specific septin-3",
  "gene": "UniProtKB:Q9UH03",
  "term_id": "GO:0031105",
  "term_label": "septin complex"
}